{
  "gene": "UniProtKB:P53672",
  "term_id": "GO:0002088",
  "gene_symbol": "CRYBA2",
  "gene_name": "Beta-crystallin A2",
  "term_label": "lens development in camera-type eye"
}